{
  "gene": "UniProtKB:Q8IV04",
  "gene_symbol": "TBC1D10C",
  "term_label": "Unknown cellular component",
  "term_id": "UNKNOWN:0003",
  "gene_name": "Carabin"
}